{
  "term_label": "focal adhesion",
  "gene_name": "Integrin beta-7",
  "gene_symbol": "ITGB7",
  "gene": "UniProtKB:P26010",
  "term_id": "GO:0005925"
}